{
  "gene": "UniProtKB:O43852",
  "gene_name": "Calumenin",
  "gene_symbol": "CALU",
  "term_label": "endoplasmic reticulum",
  "term_id": "GO:0005783"
}